{
  "term_label": "Unknown molecular function",
  "gene": "UniProtKB:Q9NXB0",
  "gene_name": "Tectonic-like complex member MKS1",
  "gene_symbol": "MKS1",
  "term_id": "UNKNOWN:0001"
}